{
  "gene_name": "Deleted in esophageal cancer 1",
  "gene": "UniProtKB:Q9P2X7",
  "term_label": "Unknown biological process",
  "term_id": "UNKNOWN:0002",
  "gene_symbol": "DELEC1"
}